{
  "gene": "UniProtKB:Q9ULL4",
  "gene_name": "Plexin-B3",
  "gene_symbol": "PLXNB3",
  "term_id": "GO:0030336",
  "term_label": "negative regulation of cell migration"
}